{
  "term_id": "UNKNOWN:0001",
  "gene_symbol": "SF3B2",
  "gene": "UniProtKB:Q13435",
  "term_label": "Unknown molecular function",
  "gene_name": "Splicing factor 3B subunit 2"
}